{
  "gene_name": "Nuclear pore complex-interacting protein family member B3",
  "term_id": "UNKNOWN:0003",
  "gene": "UniProtKB:Q92617",
  "term_label": "Unknown cellular component",
  "gene_symbol": "NPIPB3"
}